{
  "term_id": "GO:0005886",
  "gene_symbol": "SEMA5A",
  "gene": "UniProtKB:Q13591",
  "gene_name": "Semaphorin-5A",
  "term_label": "plasma membrane"
}